{
  "gene_symbol": "THEMIS2",
  "gene_name": "Protein THEMIS2",
  "gene": "UniProtKB:Q5TEJ8",
  "term_label": "Unknown molecular function",
  "term_id": "UNKNOWN:0001"
}